{
  "gene_symbol": "MAOA",
  "term_label": "mitochondrion",
  "gene_name": "Amine oxidase [flavin-containing] A",
  "gene": "UniProtKB:P21397",
  "term_id": "GO:0005739"
}